neurotransmitter receptor transport to postsynaptic membrane [GO:0098969] (biological process) Definition: The directed movement of neurotransmitter receptor to the postsynaptic membrane in transport vesicles. Sources: GOC:dos Relationships: is a type of receptor localization to synapse [GO:0097120]; is a type of neurotransmitter receptor transport to plasma membrane [GO:0098877]; is_a GO:0099072; is a type of protein localization to postsynaptic membrane [GO:1903539]; is a type of establishment of protein localization to postsynaptic membrane [GO:1903540] Subtypes: neurotransmitter receptor transport, endosome to postsynaptic membrane [GO:0098887]